cellular bud neck septin collar [GO:0032174] (cellular component) Definition: A tubular structure with flared ends, shaped like an hourglass and composed of highly ordered arrays of septin filaments, that forms at the bud neck of a dividing cell. In S. cerevisiae, this structure is located at the bud neck throughout most of the cell cycle and the septins are fixed within the structure, not exchanging with soluble septins. This septin structure acts as a scaffold for other proteins that function at the bud neck. References: PMID:16009555 Sources: GOC:krc Relationships: is a type of GO:0000399; is a type of cleavage apparatus septin structure [GO:0032161]; is a type of septin collar [GO:0032173]